{
  "gene_name": "Embryonic stem cell-related gene protein",
  "gene": "UniProtKB:Q1W209",
  "term_label": "Unknown molecular function",
  "gene_symbol": "ESRG",
  "term_id": "UNKNOWN:0001"
}